myoblast maturation involved in muscle regeneration [GO:0014914] (biological process) Sources: CL:0000056, GOC:mtg_muscle Definition: A developmental process, independent of morphogenetic (shape) change, that is required for a myoblast cell to attain its fully functional state involved in muscle regeneration. A myoblast is a mononucleate cell type that, by fusion with other myoblasts, gives rise to the myotubes that eventually develop into skeletal muscle fibers. Relationships: is a type of myoblast maturation [GO:0048628]